{
  "term_label": "Unknown cellular component",
  "gene_symbol": "FAM184B",
  "gene_name": "Protein FAM184B",
  "gene": "UniProtKB:Q9ULE4",
  "term_id": "UNKNOWN:0003"
}